{
  "term_id": "UNKNOWN:0001",
  "gene_symbol": "C11orf71",
  "term_label": "Unknown molecular function",
  "gene_name": "Uncharacterized protein C11orf71",
  "gene": "UniProtKB:Q6IPW1"
}